{
  "gene_name": "Netrin-3",
  "term_label": "RNA polymerase II cis-regulatory region sequence-specific DNA binding",
  "gene_symbol": "NTN3",
  "gene": "UniProtKB:O00634",
  "term_id": "GO:0000978"
}